symbiont-mediated perturbation of host chromatin organization [GO:0039525] (biological process) References: PMID:11483770, PMID:16687403 Sources: GOC:bf, GOC:sp Relationships: is a type of GO:0044068 Also known as: modulation by virus of host chromatin organisation, modulation of host chromatin by virus, modulation of host chromatin structure by virus, modulation by virus of host chromatin organization, regulation by virus of host chromatin organization Definition: A process in which a symbiont alters or subverts the organization of chromatin in its host. The host is defined as the larger of the organisms involved in a symbiotic interaction.